{
  "gene_symbol": "KCNQ1DN",
  "gene_name": "KCNQ1 downstream neighbor protein",
  "term_id": "UNKNOWN:0001",
  "gene": "UniProtKB:Q9H478",
  "term_label": "Unknown molecular function"
}